negative regulation of pentasaccharide transport [GO:1900361] (biological process) Also known as: down regulation of pentasaccharide transport, down-regulation of pentasaccharide transport, downregulation of pentasaccharide transport, inhibition of pentasaccharide transport Definition: Any process that stops, prevents or reduces the frequency, rate or extent of pentasaccharide transport. Subtypes: GO:1900316 Relationships: is a type of negative regulation of transport [GO:0051051]; is_a GO:1900360; negatively regulates pentasaccharide transport [GO:2001100] Sources: GOC:TermGenie, GOC:mengo_curators